{
  "gene_name": "Keratin, type I cytoskeletal 25",
  "term_id": "GO:0031069",
  "gene": "UniProtKB:Q7Z3Z0",
  "term_label": "hair follicle morphogenesis",
  "gene_symbol": "KRT25"
}